positive regulation of galactotriose transport [GO:1900293] (biological process) Also known as: up regulation of galactotriose transport, up-regulation of galactotriose transport, upregulation of galactotriose transport, activation of galactotriose transport Relationships: is a type of positive regulation of transport [GO:0051050]; is a type of regulation of galactotriose transport [GO:1900291]; positively regulates GO:2001093 Sources: GOC:TermGenie, GOC:mengo_curators Definition: Any process that activates or increases the frequency, rate or extent of galactotriose transport.